bacitracin A catabolic process [GO:1901123] (biological process) Definition: The chemical reactions and pathways resulting in the breakdown of bacitracin A. Relationships: is a type of catabolic process [GO:0009056]; is a type of amide metabolic process [GO:0043603] Sources: GOC:TermGenie, GOC:yaf, UniPathway:UPA00179 Also known as: bacitracin A breakdown, bacitracin A catabolism, bacitracin A degradation